{
  "gene_symbol": "GHRHR",
  "term_id": "GO:0008284",
  "gene": "UniProtKB:Q02643",
  "gene_name": "Growth hormone-releasing hormone receptor",
  "term_label": "positive regulation of cell population proliferation"
}